{
  "gene": "UniProtKB:Q9P2E5",
  "term_label": "glucuronosyl-N-acetylgalactosaminyl-proteoglycan 4-beta-N-acetylgalactosaminyltransferase activity",
  "gene_name": "Chondroitin sulfate glucuronyltransferase",
  "term_id": "GO:0047238",
  "gene_symbol": "CHPF2"
}